{
  "gene_name": "Small integral membrane protein 18",
  "term_label": "Unknown biological process",
  "term_id": "UNKNOWN:0002",
  "gene_symbol": "SMIM18",
  "gene": "UniProtKB:P0DKX4"
}